radial axis specification [GO:0009945] (biological process) Definition: The establishment, maintenance and elaboration of an axis that initiates at a point and radiates outward from the point. Sources: GOC:dph, GOC:go_curators, GOC:isa_complete Relationships: is a type of axis specification [GO:0009798]; is part of radial pattern formation [GO:0009956]